development of symbiont in host [GO:0044114] (biological process) Relationships: is a type of formation of structure involved in a symbiotic process [GO:0044111] Also known as: development of symbiont in host intercellular space, development of symbiont in host vascular tissue Regulation: regulated by GO:0044127; positively regulated by positive regulation of development of symbiont in host [GO:0044129]; negatively regulated by negative regulation of development of symbiont in host [GO:0044131] Note: This term partially replaces the obsolete term 'growth or development of symbiont in host ; GO:0044412'. See also 'biological process involved in interaction with host ; GO:0051701. Subtypes: dormancy entry of symbiont in host [GO:0085014], dormancy maintenance of symbiont in host [GO:0085015], dormancy exit of symbiont in host [GO:0085016], GO:0120310, procyclogenesis [GO:0120324], metacyclogenesis [GO:0140384] Sources: GOC:jl, GOC:pamgo_curators Definition: The progression of an organism from an initial condition to a later condition, occurring within the cells or tissues of the host organism. This may (but not necessarily) include a filamentous growth form, and also can include secretion of proteases and lipases to break down host tissue. The host is defined as the larger of the organisms involved in a symbiotic interaction.